{
  "term_label": "Unknown biological process",
  "gene_name": "Bromodomain adjacent to zinc finger domain protein 2B",
  "gene": "UniProtKB:Q9UIF8",
  "gene_symbol": "BAZ2B",
  "term_id": "UNKNOWN:0002"
}